{
  "term_label": "Unknown molecular function",
  "gene_name": "Neuropeptide S",
  "gene_symbol": "NPS",
  "term_id": "UNKNOWN:0001",
  "gene": "UniProtKB:P0C0P6"
}